{
  "term_id": "GO:0005634",
  "gene_name": "Homeobox protein CDX-1",
  "gene_symbol": "CDX1",
  "term_label": "nucleus",
  "gene": "UniProtKB:P47902"
}